frontonasal suture morphogenesis [GO:0097095] (biological process) Relationships: is a type of craniofacial suture morphogenesis [GO:0097094] References: PMID:12416537 Sources: GOC:pr, GOC:sl, Wikipedia:Cranial_sutures, Wikipedia:Head_and_neck_anatomy#Musculoskeletal_system Definition: The process in which the frontonasal suture, between frontal and nasal bones, is generated and organized. Also known as: nasofrontal suture morphogenesis